{
  "term_label": "nucleus",
  "gene_name": "Steroid hormone receptor ERR2",
  "gene_symbol": "ESRRB",
  "gene": "UniProtKB:O95718",
  "term_id": "GO:0005634"
}